{
  "gene_symbol": "CYLD",
  "term_id": "GO:0007346",
  "gene": "UniProtKB:Q9NQC7",
  "gene_name": "Ubiquitin carboxyl-terminal hydrolase CYLD",
  "term_label": "regulation of mitotic cell cycle"
}